{
  "term_label": "mitochondrial inner membrane",
  "gene_name": "Sideroflexin-5",
  "gene_symbol": "SFXN5",
  "gene": "UniProtKB:Q8TD22",
  "term_id": "GO:0005743"
}